regulation of epithelial to mesenchymal transition involved in endocardial cushion formation [GO:1905005] (biological process) Definition: Any process that modulates the frequency, rate or extent of epithelial to mesenchymal transition involved in endocardial cushion formation. References: PMID:18718461 Sources: GOC:BHF, GOC:TermGenie, GOC:rl, GO_REF:0000058 Relationships: is a type of regulation of cardiac epithelial to mesenchymal transition [GO:0062042]; regulates epithelial to mesenchymal transition involved in endocardial cushion formation [GO:0003198] Subtypes: negative regulation of epithelial to mesenchymal transition involved in endocardial cushion formation [GO:1905006], positive regulation of epithelial to mesenchymal transition involved in endocardial cushion formation [GO:1905007]